3alpha,7alpha,12alpha-trihydroxy-5beta-cholestanoyl-CoA 24-hydroxylase activity [GO:0033791] (molecular function) Definition: Catalysis of the reaction: (25R)-3alpha,7alpha,12alpha-trihydroxy-5beta-cholestan-26-oyl-CoA + H2O + acceptor = (24R,25R)-3alpha,7alpha,12alpha,24-tetrahydroxy-5beta-cholestan-26-oyl-CoA + reduced acceptor. Sources: EC:1.17.99.3 Also known as: (25R)-3alpha,7alpha,12alpha-trihydroxy-5beta-cholestan-26-oyl-CoA:acceptor 24-oxidoreductase (24R-hydroxylating) activity, 3alpha,7alpha,12alpha-trihydroxy-5beta-cholestan-26-oate 24-hydroxylase activity, 3alpha,7alpha,12alpha-trihydroxy-5beta-cholestanoyl-CoA oxidase activity, THC-CoA oxidase activity, THCA-CoA oxidase activity, trihydroxycoprostanoyl-CoA oxidase activity Relationships: is a type of oxidoreductase activity, acting on CH or CH2 groups [GO:0016725]